{
  "gene_symbol": "ATP1A1",
  "gene_name": "Sodium_potassium-transporting ATPase subunit alpha-1",
  "gene": "UniProtKB:P05023",
  "term_id": "GO:0006883",
  "term_label": "intracellular sodium ion homeostasis"
}